{
  "gene": "UniProtKB:Q5VWM3",
  "term_label": "cytoplasm",
  "gene_symbol": "PRAMEF18",
  "gene_name": "PRAME family member 18",
  "term_id": "GO:0005737"
}